{
  "term_label": "Unknown biological process",
  "gene_symbol": "POLR1G",
  "gene": "UniProtKB:O15446",
  "term_id": "UNKNOWN:0002",
  "gene_name": "DNA-directed RNA polymerase I subunit RPA34"
}